{
  "gene_name": "Ski-like protein",
  "gene": "UniProtKB:P12757",
  "term_id": "GO:0030514",
  "gene_symbol": "SKIL",
  "term_label": "negative regulation of BMP signaling pathway"
}